{
  "gene": "UniProtKB:P19237",
  "term_label": "cardiac muscle contraction",
  "gene_name": "Troponin I, slow skeletal muscle",
  "term_id": "GO:0060048",
  "gene_symbol": "TNNI1"
}